{
  "gene_name": "Putative trypsin-6",
  "gene_symbol": "PRSS3P2",
  "term_label": "serine-type endopeptidase activity",
  "term_id": "GO:0004252",
  "gene": "UniProtKB:Q8NHM4"
}